{
  "gene": "UniProtKB:Q9NTI5",
  "term_id": "GO:0007064",
  "gene_name": "Sister chromatid cohesion protein PDS5 homolog B",
  "gene_symbol": "PDS5B",
  "term_label": "mitotic sister chromatid cohesion"
}